{
  "gene_name": "Immunoglobulin heavy variable 2-70D",
  "gene": "UniProtKB:A0A0C4DH43",
  "gene_symbol": "IGHV2-70D",
  "term_label": "immunoglobulin mediated immune response",
  "term_id": "GO:0016064"
}